{
  "gene_name": "Dual specificity protein phosphatase 5",
  "term_id": "GO:0005737",
  "gene_symbol": "DUSP5",
  "term_label": "cytoplasm",
  "gene": "UniProtKB:Q16690"
}